{
  "gene": "UniProtKB:P11844",
  "gene_name": "Gamma-crystallin A",
  "gene_symbol": "CRYGA",
  "term_id": "UNKNOWN:0003",
  "term_label": "Unknown cellular component"
}